{
  "gene_name": "Histone-lysine N-methyltransferase EHMT1",
  "gene_symbol": "EHMT1",
  "term_label": "negative regulation of transcription by RNA polymerase II",
  "term_id": "GO:0000122",
  "gene": "UniProtKB:Q9H9B1"
}